protein demethylase activity [GO:0140457] (MF) Definition: Catalysis of the removal of a methyl group from a protein. Relationships: is a type of GO:0032451; is_a GO:0140096 Subtypes: histone demethylase activity [GO:0032452] References: PMID:24498420, PMID:28360925